{
  "gene_symbol": "ZNF331",
  "gene": "UniProtKB:Q9NQX6",
  "term_label": "Unknown cellular component",
  "term_id": "UNKNOWN:0003",
  "gene_name": "Zinc finger protein 331"
}